{
  "gene": "UniProtKB:Q8N7M2",
  "gene_name": "Zinc finger protein 283",
  "gene_symbol": "ZNF283",
  "term_label": "nucleus",
  "term_id": "GO:0005634"
}